metestrus [GO:0060210] (biological process) Sources: GOC:dph, ISBN:0721662544 Note: Note that this term should not be used for direct annotation. If you are trying to make an annotation to x phase, it is likely that the correct annotation is 'regulation of x/y phase transition' or to a process which occurs during the reported phase. To capture the phase when a specific location or process is observed, the phase term can be used in an annotation extension (PMID:24885854) applied to a cellular component term (with the relation exists_during) or a biological process term (with the relation happens_during). Definition: The estrous cycle phase in which there is subsiding follicular function. Relationships: is a type of estrous cycle phase [GO:0060206]